{
  "gene": "UniProtKB:P0DW11",
  "gene_symbol": "TAF11L6",
  "term_id": "GO:0051123",
  "gene_name": "TATA-box-binding protein-associated factor 11-like protein 6",
  "term_label": "RNA polymerase II preinitiation complex assembly"
}